secretion by tissue [GO:0032941] (biological process) Subtypes: pancreatic juice secretion [GO:0030157], cerebrospinal fluid secretion [GO:0033326], saliva secretion [GO:0046541], milk ejection reflex [GO:0060156], tear secretion [GO:0070075], mucus secretion [GO:0070254], sweat secretion [GO:0160269] Definition: The controlled release of a substance by a tissue. Also known as: tissue secretion, expulsion of gland contents Relationships: is a type of multicellular organismal process [GO:0032501]; is a type of secretion [GO:0046903] Sources: GOC:mah